zeatin biosynthetic process [GO:0033398] (biological process) Relationships: is a type of cytokinin biosynthetic process [GO:0009691]; is a type of purine-containing compound biosynthetic process [GO:0072522] Subtypes: GO:0033465, GO:0033466 Also known as: zeatin anabolism, zeatin biosynthesis, zeatin formation, zeatin synthesis Definition: The chemical reactions and pathways resulting in the formation of zeatin, 2-methyl-4-(9H-purin-6-ylamino)but-2-en-1-ol. Sources: GOC:mah